dense core granule exocytosis [GO:1990504] (biological process) Also known as: dense core vesicle exocytosis References: PMID:17553987, PMID:24653208 Sources: GOC:kmv Regulation: regulated by GO:1905413; RO_0002212 by negative regulation of dense core granule exocytosis [GO:1905414]; positively regulated by positive regulation of dense core granule exocytosis [GO:1905415] Definition: The secretion of molecules (e.g. neuropeptides, insulin-related peptides or neuromodulators such as serotonin and dopamine) contained within a membrane-bounced dense core granule by fusion of the granule with the plasma membrane of a cell in response to increased cytosolic calcium levels. Subtypes: neuronal dense core vesicle exocytosis [GO:0099011] Relationships: is a type of calcium-ion regulated exocytosis [GO:0017156]; is a type of dense core granule localization [GO:0032253]; is a type of establishment of vesicle localization [GO:0051650]